{
  "term_label": "immune receptor activity",
  "gene_symbol": "KIR2DL2",
  "gene_name": "Killer cell immunoglobulin-like receptor 2DL2",
  "gene": "UniProtKB:P43627",
  "term_id": "GO:0140375"
}